{
  "gene_name": "Bestrophin-2",
  "gene": "UniProtKB:Q8NFU1",
  "term_id": "GO:0005886",
  "gene_symbol": "BEST2",
  "term_label": "plasma membrane"
}